{
  "gene_symbol": "GUCY2F",
  "term_label": "visual perception",
  "gene_name": "Retinal guanylyl cyclase 2",
  "term_id": "GO:0007601",
  "gene": "UniProtKB:P51841"
}